{
  "term_id": "GO:0051082",
  "gene": "UniProtKB:Q96NT0",
  "gene_symbol": "VMA22",
  "term_label": "unfolded protein binding",
  "gene_name": "Coiled-coil domain-containing protein 115"
}